nucleotide transport [GO:0006862] (biological process) Relationships: is a type of organophosphate ester transport [GO:0015748]; is a type of GO:0015931 Sources: ISBN:0198506732 Definition: The directed movement of a nucleotide, any compound consisting of a nucleoside that is esterified with (ortho)phosphate, into, out of or within a cell. Subtypes: pyrimidine nucleotide transport [GO:0006864], purine nucleotide transport [GO:0015865], GO:0015883, nicotinamide mononucleotide transport [GO:0015890], deoxynucleotide transport [GO:0030302], cyclic nucleotide transport [GO:0070729], nucleotide transmembrane transport [GO:1901679]